{
  "term_id": "GO:0004888",
  "term_label": "transmembrane signaling receptor activity",
  "gene_symbol": "KIR3DL1",
  "gene_name": "Killer cell immunoglobulin-like receptor 3DL1",
  "gene": "UniProtKB:P43629"
}